{
  "gene": "UniProtKB:A6NJB7",
  "term_id": "UNKNOWN:0002",
  "gene_name": "Proline-rich protein 19",
  "term_label": "Unknown biological process",
  "gene_symbol": "PRR19"
}